{
  "gene_name": "NACHT, LRR and PYD domains-containing protein 1",
  "term_label": "inflammatory response",
  "term_id": "GO:0006954",
  "gene_symbol": "NLRP1",
  "gene": "UniProtKB:Q9C000"
}